carboxymethylenebutenolidase activity [GO:0008806] (molecular function) Relationships: is a type of carboxylic ester hydrolase activity [GO:0052689] Sources: EC:3.1.1.45 Also known as: 4-carboxymethylenebut-2-en-4-olide lactonohydrolase activity, carboxymethylene butenolide hydrolase activity, dienelactone hydrolase activity, maleylacetate enol-lactonase activity Definition: Catalysis of the reaction: 4-carboxymethylenebut-2-en-4-olide + H2O = 4 oxohex-2-enedioate.